{
  "gene": "UniProtKB:Q5T681",
  "gene_symbol": "C10orf62",
  "gene_name": "Uncharacterized protein C10orf62",
  "term_id": "UNKNOWN:0003",
  "term_label": "Unknown cellular component"
}